{
  "gene_name": "Selenocysteine insertion sequence-binding protein 2-like",
  "gene": "UniProtKB:Q93073",
  "term_label": "mRNA 3'-UTR binding",
  "gene_symbol": "SECISBP2L",
  "term_id": "GO:0003730"
}